{
  "term_id": "UNKNOWN:0003",
  "term_label": "Unknown cellular component",
  "gene_name": "Sushi domain-containing protein 1",
  "gene": "UniProtKB:Q6UWL2",
  "gene_symbol": "SUSD1"
}